agmatine:putrescine antiporter activity [GO:0043861] (molecular function) Definition: Catalysis of the reaction: agmatine(out) + putrescine(in) = agmatine(in) + putrescine(out). References: PMID:17028272 Sources: GOC:jl Also known as: agmatine-putrescine antiporter activity, agmatine/putrescine antiporter activity Relationships: is a type of antiporter activity [GO:0015297]; is a type of putrescine transmembrane transporter activity [GO:0015489]